interleukin-4-dependent isotype switching to IgE isotypes [GO:0035708] (biological process) Definition: The switching of activated B cells from IgM biosynthesis to IgE biosynthesis, accomplished through a recombination process involving an intrachromosomal deletion between switch regions that reside 5' of the IgM and IgE constant region gene segments in the immunoglobulin heavy chain locus, that is dependent on the activity of interleukin 4 (IL-4). Relationships: is a type of GO:0048289 References: PMID:12496423 Sources: GOC:BHF Regulation: regulated by regulation of interleukin-4-dependent isotype switching to IgE isotypes [GO:2000571]; RO_0002213 by positive regulation of interleukin-4-dependent isotype switching to IgE isotypes [GO:2000572] Also known as: IL-4-dependent isotype switching to IgE isotypes